{
  "term_id": "GO:1904862",
  "gene_symbol": "GABRA5",
  "gene_name": "Gamma-aminobutyric acid receptor subunit alpha-5",
  "term_label": "inhibitory synapse assembly",
  "gene": "UniProtKB:P31644"
}